{
  "gene_symbol": "MTMR12",
  "gene_name": "Myotubularin-related protein 12",
  "term_label": "cytoplasm",
  "gene": "UniProtKB:Q9C0I1",
  "term_id": "GO:0005737"
}